{
  "gene": "UniProtKB:Q6FI81",
  "gene_name": "Anamorsin",
  "term_id": "GO:0016226",
  "term_label": "iron-sulfur cluster assembly",
  "gene_symbol": "CIAPIN1"
}